{
  "term_label": "ATPase-coupled intramembrane lipid transporter activity",
  "gene": "UniProtKB:Q9P241",
  "gene_symbol": "ATP10D",
  "term_id": "GO:0140326",
  "gene_name": "Phospholipid-transporting ATPase VD"
}